{
  "gene_name": "FK506-binding protein 15",
  "gene_symbol": "FKBP15",
  "term_id": "GO:0030426",
  "gene": "UniProtKB:Q5T1M5",
  "term_label": "growth cone"
}